histone H3K79 monomethyltransferase activity [GO:0120505] (molecular function) Relationships: is a type of histone H3K79 methyltransferase activity [GO:0031151] Definition: Catalysis of the reaction: L-lysyl79-[histone H3] + S-adenosyl-L-methionine = H+ + N6-methyl-L-lysyl79-[histone H3] + S-adenosyl-L-homocysteine. Note: Comment: Note that the residue position corresponds to the canonical human H3 histone (UniProtKB:P84243); this residue is conserved across all eukaryotes. Residue 1 is the first residue following removal of the initiating Methionine (Met). Note that each histone is encoded by multiple genes, and sequences may vary across different genes within an organism. References: PMID:14732680, PMID:15371351 Sources: RHEA:60332